{
  "gene_symbol": "H2BC9",
  "gene_name": "Histone H2B type 1-H",
  "gene": "UniProtKB:Q93079",
  "term_id": "GO:0061844",
  "term_label": "antimicrobial humoral immune response mediated by antimicrobial peptide"
}